carbohydrate binding [GO:0030246] (molecular function) Also known as: sugar binding, selectin Definition: Binding to a carbohydrate, which includes monosaccharides, oligosaccharides and polysaccharides as well as substances derived from monosaccharides by reduction of the carbonyl group (alditols), by oxidation of one or more hydroxy groups to afford the corresponding aldehydes, ketones, or carboxylic acids, or by replacement of one or more hydroxy group(s) by a hydrogen atom. Cyclitols are generally not regarded as carbohydrates. Subtypes: GO:0030247, GO:0048029, oligosaccharide binding [GO:0070492], calcium-dependent carbohydrate binding [GO:0120153] Relationships: is a type of binding [GO:0005488] Sources: GOC:mah